5-O-(4-coumaroyl)-D-quinate 3'-monooxygenase activity [GO:0047083] (MF) Sources: EC:1.14.14.96, MetaCyc:1.14.13.36-RXN Definition: Catalysis of the reaction: O2 + NADPH + H+ + trans-5-O-(4-coumaroyl)-D-quinate = H2O + NADP+ + trans-5-O-caffeoyl-D-quinate. Relationships: is a type of GO:0016709 Also known as: 5-O-(4-coumaroyl)-D-quinate/shikimate 3'-hydroxylase activity, coumaroylquinate(coumaroylshikimate) 3'-monooxygenase activity, trans-5-O-(4-coumaroyl)-D-quinate,NADPH:oxygen oxidoreductase (3'-hydroxylating)